pyrimidine deoxyribonucleoside biosynthetic process [GO:0046126] (BP) Definition: The chemical reactions and pathways resulting in the formation of any one of a family of organic molecules consisting of a pyrimidine base covalently bonded to a sugar deoxyribose (a deoxyribonucleoside). Sources: GOC:ai Relationships: is a type of deoxyribonucleoside biosynthetic process [GO:0046120]; is a type of GO:0046125; is a type of GO:0046134 Subtypes: pyrimidine deoxyribonucleoside salvage [GO:0043099], deoxycytidine biosynthetic process [GO:0046093], deoxyuridine biosynthetic process [GO:0046097], thymidine biosynthetic process [GO:0046105] Also known as: pyrimidine deoxyribonucleoside anabolism, pyrimidine deoxyribonucleoside biosynthesis, pyrimidine deoxyribonucleoside formation, pyrimidine deoxyribonucleoside synthesis